plasma membrane raft organization [GO:0044857] (biological process) Sources: GOC:jl Subtypes: plasma membrane raft assembly [GO:0044854] Definition: A process that is carried out at the cellular level which results in the assembly, arrangement of constituent parts, or disassembly of plasma membrane rafts. Relationships: is a type of GO:0031579; BFO_0000050 plasma membrane organization [GO:0007009]